{
  "gene_symbol": "CEMP1",
  "gene": "UniProtKB:Q6PRD7",
  "term_id": "GO:0005634",
  "term_label": "nucleus",
  "gene_name": "Cementoblastoma-derived protein 1"
}